{
  "gene_symbol": "PRMT9",
  "gene_name": "Protein arginine N-methyltransferase 9",
  "term_label": "chromatin remodeling",
  "term_id": "GO:0006338",
  "gene": "UniProtKB:Q6P2P2"
}